{
  "gene_symbol": "RUSC2",
  "term_label": "Unknown biological process",
  "term_id": "UNKNOWN:0002",
  "gene": "UniProtKB:Q8N2Y8",
  "gene_name": "AP-4 complex accessory subunit RUSC2"
}